{
  "term_label": "fructose transmembrane transporter activity",
  "gene_name": "Solute carrier family 2, facilitated glucose transporter member 5",
  "gene_symbol": "SLC2A5",
  "gene": "UniProtKB:P22732",
  "term_id": "GO:0005353"
}